{
  "gene_name": "SLIT and NTRK-like protein 2",
  "term_id": "GO:0098978",
  "term_label": "glutamatergic synapse",
  "gene": "UniProtKB:Q9H156",
  "gene_symbol": "SLITRK2"
}